{
  "gene_name": "Ras-related C3 botulinum toxin substrate 2",
  "term_label": "plasma membrane",
  "gene_symbol": "RAC2",
  "gene": "UniProtKB:P15153",
  "term_id": "GO:0005886"
}